{
  "gene_symbol": "TBX4",
  "gene_name": "T-box transcription factor TBX4",
  "term_label": "angiogenesis",
  "term_id": "GO:0001525",
  "gene": "UniProtKB:P57082"
}